negative regulation of cell cycle G2/M phase transition [GO:1902750] (biological process) Definition: Any signaling pathway that decreases or inhibits the activity of a cell cycle cyclin-dependent protein kinase to modulate the switch from G2 phase to M phase of the cell cycle. Sources: GOC:TermGenie, GOC:jl, GO_REF:0000058 Relationships: is a type of negative regulation of cell cycle phase transition [GO:1901988]; is a type of regulation of cell cycle G2/M phase transition [GO:1902749]; negatively regulates cell cycle G2/M phase transition [GO:0044839] Subtypes: GO:0010972, negative regulation of G2/MI transition of meiotic cell cycle [GO:0110031] Also known as: down regulation of cell cycle G2/M phase transition, down-regulation of cell cycle G2/M phase transition, downregulation of cell cycle G2/M phase transition, inhibition of cell cycle G2/M phase transition